copper-dependent protein binding [GO:0032767] (molecular function) References: PMID:16884690 Sources: GOC:ecd Definition: Binding to a protein or protein complex, in the presence of copper. Relationships: is_a GO:0005515